chemoattraction of dopaminergic neuron axon [GO:0036516] (biological process) Definition: The process in which a dopaminergic neuron growth cone is directed to a specific target site in response to an attractive chemical signal. Relationships: is a type of chemoattraction of axon [GO:0061642]; is part of dopaminergic neuron axon guidance [GO:0036514] Also known as: chemoattraction of DA axon, chemoattraction of dopaminergic axon References: PMID:21106844 Sources: GOC:PARL, GOC:bf